alkylated DNA binding [GO:0032131] (MF) Relationships: is a type of damaged DNA binding [GO:0003684] Sources: GOC:mah Subtypes: GO:0032132 Definition: Binding to an alkylated residue in DNA.